{
  "gene_name": "Src kinase-associated phosphoprotein 2",
  "gene": "UniProtKB:O75563",
  "term_id": "UNKNOWN:0001",
  "term_label": "Unknown molecular function",
  "gene_symbol": "SKAP2"
}